{
  "gene": "UniProtKB:Q8NB66",
  "gene_symbol": "UNC13C",
  "term_id": "GO:0031594",
  "term_label": "neuromuscular junction",
  "gene_name": "Protein unc-13 homolog C"
}